{
  "term_label": "oligosaccharide biosynthetic process",
  "gene_name": "Beta-1,3-galactosyltransferase 1",
  "gene": "UniProtKB:Q9Y5Z6",
  "gene_symbol": "B3GALT1",
  "term_id": "GO:0009312"
}